{
  "gene_name": "NLR family CARD domain-containing protein 3",
  "term_id": "UNKNOWN:0001",
  "term_label": "Unknown molecular function",
  "gene_symbol": "NLRC3",
  "gene": "UniProtKB:Q7RTR2"
}